protein localization to microtubule plus-end [GO:1904825] (biological process) Definition: A process in which a protein is transported to, or maintained in, a location at a microtubule plus-end. References: PMID:24039245 Sources: GOC:TermGenie, GO_REF:0000087 Also known as: protein localisation to microtubule plus-end Relationships: is a type of GO:1905725 Subtypes: GO:1904518